alpha-2A adrenergic receptor binding [GO:0031694] (molecular function) Relationships: is a type of adrenergic receptor binding [GO:0031690] Sources: GOC:mah, GOC:nln Also known as: alpha-2A adrenergic receptor ligand Definition: Binding to an alpha-2A adrenergic receptor.